{
  "term_id": "GO:0003690",
  "term_label": "double-stranded DNA binding",
  "gene_name": "Histone H1.8",
  "gene": "UniProtKB:Q8IZA3",
  "gene_symbol": "H1-8"
}